{
  "gene_name": "BTB_POZ domain-containing protein KCTD8",
  "gene_symbol": "KCTD8",
  "gene": "UniProtKB:Q6ZWB6",
  "term_label": "Unknown molecular function",
  "term_id": "UNKNOWN:0001"
}